protein-disulfide reductase [NAD(P)H] activity [GO:0047134] (molecular function) Relationships: is a type of protein-disulfide reductase activity [GO:0015035]; is a type of oxidoreductase activity, acting on a sulfur group of donors, NAD(P) as acceptor [GO:0016668] Sources: EC:1.8.1.8 Subtypes: GO:0004791 Also known as: protein-disulfide reductase activity, protein-disulphide reductase activity, protein disulfide reductase (NAD(P)H) activity, protein-disulfide reductase (NAD(P)) activity, NAD(P)H:protein-disulfide oxidoreductase activity, disulfide reductase activity, insulin-glutathione transhydrogenase activity, protein disulfide reductase activity, protein disulphide reductase activity Definition: Catalysis of the reaction: protein-dithiol + NAD(P)+ = protein-disulfide + NAD(P)H + H+.